positive regulation of response to toluene [GO:1901456] (biological process) Sources: GOC:TermGenie, GOC:mengo_curators Also known as: up regulation of response to toluene, up-regulation of response to toluene, upregulation of response to toluene, activation of response to toluene Definition: Any process that activates or increases the frequency, rate or extent of response to toluene. Relationships: is a type of positive regulation of response to stimulus [GO:0048584]; is a type of GO:1901454; RO_0002213 response to toluene [GO:1901424]